{
  "gene_name": "Structural maintenance of chromosomes protein 2",
  "gene_symbol": "SMC2",
  "gene": "UniProtKB:O95347",
  "term_label": "condensin complex",
  "term_id": "GO:0000796"
}